{
  "gene": "UniProtKB:O95402",
  "term_label": "regulation of transcription by RNA polymerase II",
  "term_id": "GO:0006357",
  "gene_symbol": "MED26",
  "gene_name": "Mediator of RNA polymerase II transcription subunit 26"
}